{
  "gene_name": "Saitohin",
  "term_id": "UNKNOWN:0003",
  "term_label": "Unknown cellular component",
  "gene_symbol": "STH",
  "gene": "UniProtKB:Q8IWL8"
}